{
  "term_id": "GO:0004521",
  "gene": "UniProtKB:Q7KZF4",
  "gene_symbol": "SND1",
  "term_label": "RNA endonuclease activity",
  "gene_name": "Staphylococcal nuclease domain-containing protein 1"
}